{
  "gene_name": "ERC protein 2",
  "term_label": "structural constituent of presynaptic active zone",
  "gene_symbol": "ERC2",
  "gene": "UniProtKB:O15083",
  "term_id": "GO:0098882"
}